sucrose catabolic process [GO:0005987] (biological process) Sources: GOC:go_curators Also known as: sucrose breakdown, sucrose catabolism, sucrose degradation Definition: The chemical reactions and pathways resulting in the breakdown of sucrose, the disaccharide fructofuranosyl-glucopyranoside. Relationships: is a type of sucrose metabolic process [GO:0005985]; is a type of disaccharide catabolic process [GO:0046352] Subtypes: sucrose catabolic process via 3'-ketosucrose [GO:0019574], sucrose catabolic process to fructose-6-phosphate and glucose-6-phosphate [GO:0036008], GO:0061704, GO:0061705